{
  "term_id": "GO:0000774",
  "term_label": "adenyl-nucleotide exchange factor activity",
  "gene_name": "BAG family molecular chaperone regulator 4",
  "gene_symbol": "BAG4",
  "gene": "UniProtKB:O95429"
}